{
  "term_label": "heart development",
  "gene_name": "Lysine-specific demethylase 6A",
  "gene": "UniProtKB:O15550",
  "gene_symbol": "KDM6A",
  "term_id": "GO:0007507"
}